ATPase-coupled L-glutamine transmembrane transporter activity [GO:0015599] (molecular function) Also known as: ATPase-coupled glutamine transmembrane transporter activity, glutamine porter activity, glutamine-importing ATPase activity Relationships: is a type of L-glutamine transmembrane transporter activity [GO:0015186]; is a type of ATPase-coupled polar amino acid-transporter activity [GO:0015426]; is a type of GO:0033284 Definition: Enables the transfer of a solute or solutes from one side of a membrane to the other according to the reaction: L-glutamine(out) + ATP + H2O = L-glutamine(in) + ADP + phosphate + H+. Sources: RHEA:29895